cerebellar granule cell precursor proliferation [GO:0021930] (biological process) Definition: The multiplication or reproduction of neuroblasts that will give rise to granule cells. A granule cell is a glutamatergic interneuron found in the cerebellar cortex. Regulation: regulated by GO:0021936; positively regulated by positive regulation of cerebellar granule cell precursor proliferation [GO:0021940]; negatively regulated by negative regulation of cerebellar granule cell precursor proliferation [GO:0021941] Relationships: is a type of cell proliferation in external granule layer [GO:0021924] References: PMID:15157725 Sources: GOC:cls, GOC:dgh, GOC:dph, GOC:jid, GO_REF:0000021